sinapate biosynthetic process [GO:0033497] (biological process) Sources: GOC:mah Also known as: sinapate anabolism, sinapate biosynthesis, sinapate formation, sinapate synthesis Definition: The chemical reactions and pathways resulting in the formation of sinapate, (2E)-3-(4-hydroxy-3,5-dimethoxyphenyl)prop-2-enoate. Relationships: is a type of phenylpropanoid biosynthetic process [GO:0009699]; is a type of benzene-containing compound metabolic process [GO:0042537]; is a type of GO:0046189; is a type of monocarboxylic acid biosynthetic process [GO:0072330]; is a type of olefinic compound biosynthetic process [GO:0120255]; is a type of ether biosynthetic process [GO:1901503]